{
  "term_id": "GO:0004180",
  "term_label": "carboxypeptidase activity",
  "gene_name": "Putative uncharacterized protein ENSP00000334305",
  "gene": "UniProtKB:Q3C1V9",
  "gene_symbol": "Q3C1V9"
}